{
  "gene_name": "Mitochondrial amidoxime reducing component 2",
  "gene": "UniProtKB:Q969Z3",
  "term_id": "GO:0030151",
  "term_label": "molybdenum ion binding",
  "gene_symbol": "MTARC2"
}